{
  "gene_name": "Target of rapamycin complex subunit LST8",
  "term_label": "TOR signaling",
  "term_id": "GO:0031929",
  "gene": "UniProtKB:Q9BVC4",
  "gene_symbol": "MLST8"
}